{
  "gene_symbol": "TNPO2",
  "term_label": "nuclear localization sequence binding",
  "gene": "UniProtKB:O14787",
  "term_id": "GO:0008139",
  "gene_name": "Transportin-2"
}